{
  "term_id": "GO:0005829",
  "gene_symbol": "CSNK2A3",
  "term_label": "cytosol",
  "gene_name": "Casein kinase II subunit alpha 3",
  "gene": "UniProtKB:Q8NEV1"
}